propionate kinase activity [GO:0008980] (molecular function) Sources: EC:2.7.2.15 Also known as: ATP:propanoate phosphotransferase activity, propanoate kinase activity, PduW, TdcD Definition: Catalysis of the reaction: ATP + propanoate = ADP + propanoyl phosphate. Relationships: is a type of kinase activity [GO:0016301]; is a type of phosphotransferase activity, carboxyl group as acceptor [GO:0016774]